2-oxobutyrate catabolic process [GO:0019606] (biological process) Definition: The chemical reactions and pathways resulting in the breakdown of 2-oxobutyrate, the anion of the organic acid 2-oxobutyric acid, which contains a ketone group on carbon 2. Also known as: 2-oxobutyrate breakdown, 2-oxobutyrate catabolism, 2-oxobutyrate degradation, alpha-ketobutyrate catabolic process, alpha-ketobutyrate catabolism Sources: ISBN:0198506732 Relationships: is a type of short-chain fatty acid catabolic process [GO:0019626]